postsynaptic dense core vesicle exocytosis [GO:0150038] (biological process) Regulation: regulated by GO:0150044 References: PMID:19448629 Sources: GOC:aruk, GOC:bc Relationships: is a type of vesicle-mediated transport in synapse [GO:0099003]; is a type of neuronal dense core vesicle exocytosis [GO:0099011]; occurs in GO:0098794 Definition: The secretion of molecules (e.g. neuropeptides, insulin-related peptides or neuromodulators such as serotonin and dopamine) contained within a postsynaptic dense core vesicle by fusion of the granule with the plasma membrane of the postsynapse in response to increased cytosolic calcium levels.